paranodal junction assembly [GO:0030913] (biological process) References: PMID:14715942 Relationships: is a type of cell-cell junction assembly [GO:0007043]; is a type of cellular component assembly involved in morphogenesis [GO:0010927]; is part of myelin assembly [GO:0032288] Definition: Formation of the junction between an axon and the glial cell that forms the myelin sheath. Paranodal junctions form at each paranode, i.e. at the ends of the unmyelinated nodes of Ranvier. Also known as: paranodal axoglial junction formation, paranodal junction biosynthesis, paranodal junction formation